N6-methyladenosine-containing RNA reader activity [GO:1990247] (MF) References: PMID:22575960, PMID:24284625 Also known as: N6-methyladenosine-containing RNA binding Relationships: is a type of protein-RNA adaptor activity [GO:0140517]; has part RNA binding [GO:0003723] Definition: A protein adaptor that recognizes and binds an RNA molecule modified by N6-methyladenosine (m6A), a modification present at internal sites of mRNAs and some non-coding RNAs.